{
  "gene": "UniProtKB:A0A075B6Z4",
  "term_label": "Unknown cellular component",
  "gene_symbol": "TRDJ4",
  "term_id": "UNKNOWN:0003",
  "gene_name": "T cell receptor delta joining 4 (Fragment)"
}